protein carboxylation [GO:0018214] (BP) Sources: GOC:ai Relationships: is a type of protein modification process [GO:0036211] Subtypes: peptidyl-glutamic acid carboxylation [GO:0017187] Definition: The addition of a carboxy group to a protein amino acid. Also known as: protein amino acid carboxylation